{
  "gene_name": "Transmembrane protein 151B",
  "term_id": "UNKNOWN:0001",
  "gene_symbol": "TMEM151B",
  "term_label": "Unknown molecular function",
  "gene": "UniProtKB:Q8IW70"
}